{
  "term_id": "GO:0003677",
  "term_label": "DNA binding",
  "gene": "UniProtKB:Q99877",
  "gene_symbol": "H2BC15",
  "gene_name": "Histone H2B type 1-N"
}